{
  "gene": "UniProtKB:Q9UIL8",
  "term_id": "UNKNOWN:0001",
  "term_label": "Unknown molecular function",
  "gene_symbol": "PHF11",
  "gene_name": "PHD finger protein 11"
}